{
  "gene_symbol": "DLG5",
  "gene_name": "Disks large homolog 5",
  "term_id": "GO:0035331",
  "term_label": "negative regulation of hippo signaling",
  "gene": "UniProtKB:Q8TDM6"
}